{
  "term_label": "chemotaxis",
  "gene": "UniProtKB:Q99788",
  "gene_symbol": "CMKLR1",
  "gene_name": "Chemerin-like receptor 1",
  "term_id": "GO:0006935"
}